{
  "gene_symbol": "GLT8D1",
  "gene_name": "Glycosyltransferase 8 domain-containing protein 1",
  "term_label": "Unknown biological process",
  "gene": "UniProtKB:Q68CQ7",
  "term_id": "UNKNOWN:0002"
}